{
  "gene_symbol": "CDC42",
  "gene_name": "Cell division control protein 42 homolog",
  "term_label": "endocytosis",
  "term_id": "GO:0006897",
  "gene": "UniProtKB:P60953"
}